{
  "term_label": "phospholipase C-activating G protein-coupled receptor signaling pathway",
  "gene_name": "Putative G-protein coupled receptor GPR32P1",
  "term_id": "GO:0007200",
  "gene_symbol": "GPR32P1",
  "gene": "UniProtKB:Q8NGA4"
}